{
  "gene_symbol": "CDADC1",
  "term_label": "Unknown biological process",
  "gene_name": "Cytidine and dCMP deaminase domain-containing protein 1",
  "gene": "UniProtKB:Q9BWV3",
  "term_id": "UNKNOWN:0002"
}